{
  "gene": "UniProtKB:X6R8D5",
  "gene_symbol": "GUCA1ANB",
  "term_label": "Unknown cellular component",
  "gene_name": "Putative uncharacterized protein GUCA1ANB",
  "term_id": "UNKNOWN:0003"
}